{
  "gene": "UniProtKB:Q8TET4",
  "term_id": "GO:0006491",
  "gene_name": "Neutral alpha-glucosidase C",
  "term_label": "N-glycan processing",
  "gene_symbol": "GANC"
}